galactinol-sucrose galactosyltransferase activity [GO:0047274] (molecular function) Definition: Catalysis of the reaction: sucrose + 1-alpha-D-galactosyl-myo-inositol = raffinose + myo-inositol. Relationships: is a type of GO:0008378 Sources: EC:2.4.1.82, MetaCyc:2.4.1.82-RXN Also known as: galactinol:sucrose 6-galactosyl transferase activity, galactosyltransferase, galactinol-sucrose, raffinose synthase activity, 1-alpha-D-galactosyl-myo-inositol:sucrose 6-alpha-D-galactosyltransferase activity, alpha-D-galactosyl-(1->3)-myo-inositol:sucrose 6-alpha-D-galactosyltransferase activity